{
  "gene_symbol": "OPN1LW",
  "gene": "UniProtKB:P04000",
  "term_id": "GO:0008020",
  "term_label": "G protein-coupled photoreceptor activity",
  "gene_name": "Long-wave-sensitive opsin 1"
}